{
  "term_label": "mRNA binding",
  "gene": "UniProtKB:Q15415",
  "gene_symbol": "RBMY1F",
  "gene_name": "RNA-binding motif protein, Y chromosome, family 1 member F_J",
  "term_id": "GO:0003729"
}